response to indole-3-methanol [GO:0071680] (biological process) Also known as: response to indole-3-carbinol Sources: GOC:mah, GOC:yaf Subtypes: GO:0071681 Definition: Any process that results in a change in state or activity of a cell or an organism (in terms of movement, secretion, enzyme production, gene expression, etc.) as a result of an indole-3-methanol stimulus. Relationships: is a type of GO:0097305; is a type of response to nitrogen compound [GO:1901698]